{
  "term_id": "GO:0035267",
  "gene_symbol": "KAT8",
  "gene": "UniProtKB:Q9H7Z6",
  "term_label": "NuA4 histone acetyltransferase complex",
  "gene_name": "Histone acetyltransferase KAT8"
}